{
  "gene": "UniProtKB:Q9BZL4",
  "term_label": "enzyme inhibitor activity",
  "term_id": "GO:0004857",
  "gene_symbol": "PPP1R12C",
  "gene_name": "Protein phosphatase 1 regulatory subunit 12C"
}